{
  "term_label": "cholesterol monooxygenase (side-chain-cleaving) activity",
  "term_id": "GO:0008386",
  "gene": "UniProtKB:P05108",
  "gene_name": "Cholesterol side-chain cleavage enzyme, mitochondrial",
  "gene_symbol": "CYP11A1"
}